{
  "gene_symbol": "FCRLB",
  "term_label": "cell surface receptor signaling pathway",
  "term_id": "GO:0007166",
  "gene": "UniProtKB:Q6BAA4",
  "gene_name": "Fc receptor-like B"
}